{
  "gene": "UniProtKB:Q15652",
  "term_label": "regulation of transcription by RNA polymerase II",
  "gene_symbol": "JMJD1C",
  "term_id": "GO:0006357",
  "gene_name": "Probable JmjC domain-containing histone demethylation protein 2C"
}